{
  "gene_name": "Vacuolar protein sorting-associated protein 52 homolog",
  "gene_symbol": "VPS52",
  "term_id": "GO:0042147",
  "term_label": "retrograde transport, endosome to Golgi",
  "gene": "UniProtKB:Q8N1B4"
}